smoothened signaling pathway involved in spinal cord motor neuron cell fate specification [GO:0021776] (biological process) Also known as: hedgehog signaling pathway involved in spinal cord motor neuron cell fate specification, hh signaling pathway involved in spinal cord motor neuron cell fate specification, smoothened signalling pathway involved in spinal cord motor neuron cell fate specification Definition: The series of molecular signals initiated by binding of a ligand to the transmembrane receptor smoothened in a precursor cell in the spinal cord that contributes to the process of a precursor cell becoming capable of differentiating autonomously into a motor neuron in an environment that is neutral with respect to the developmental pathway. References: PMID:15936325 Sources: GOC:cls, GOC:dgh, GOC:dph, GOC:jid, GO_REF:0000021 Relationships: is a type of smoothened signaling pathway involved in ventral spinal cord patterning [GO:0021910]; is part of GO:0021520